glycogenin glucosyltransferase activity [GO:0008466] (molecular function) Definition: Catalysis of the reaction: UDP-glucose + glycogenin = UDP + glucosylglycogenin. This first reaction is a self glucosylation. Further UDP-glucose goups are added to the [1,4-alpha-D-glucosyl](n) group of glycogenin until a length of about 5-13 residues. Sources: EC:2.4.1.186 Also known as: 1,4alpha-glucan-protein synthase (UDP-forming) activity, alpha-1,4-glucan-protein synthase (UDP-forming) activity, UDP-alpha-D-glucose:glycogenin alpha-D-glucosyltransferase activity, UDP-glucose:glycogenin glucosyltransferase activity, glycogenin activity, priming glucosyltransferase activity Relationships: is a type of UDP-glucosyltransferase activity [GO:0035251]